{
  "gene": "UniProtKB:P04155",
  "term_id": "GO:0005615",
  "gene_symbol": "TFF1",
  "gene_name": "Trefoil factor 1",
  "term_label": "extracellular space"
}